O-malonyltransferase activity [GO:0050736] (MF) Definition: Catalysis of the transfer of a malonyl group to an oxygen atom on the acceptor molecule. Subtypes: isoflavone-7-O-beta-glucoside 6''-O-malonyltransferase activity [GO:0047164], GO:0047165 Relationships: is a type of O-acyltransferase activity [GO:0008374]; is_a GO:0016420 Sources: GOC:ai